{
  "term_id": "GO:0034706",
  "gene_name": "Amiloride-sensitive sodium channel subunit delta",
  "gene": "UniProtKB:P51172",
  "term_label": "sodium channel complex",
  "gene_symbol": "SCNN1D"
}